chitin catabolic process [GO:0006032] (biological process) Also known as: beta-1,4-linked N-acetylglucosamine catabolic process, beta-1,4-linked N-acetylglucosamine catabolism, chitin breakdown, chitin catabolism, chitin degradation Sources: GOC:jl, ISBN:0198506732 Subtypes: chitin catabolic process to fructose 6-phosphate via glucosamine [GO:0052776] Relationships: is a type of aminoglycan catabolic process [GO:0006026]; is a type of chitin metabolic process [GO:0006030]; is a type of GO:1901072 Definition: The chemical reactions and pathways resulting in the breakdown of chitin, a linear polysaccharide consisting of beta-(1->4)-linked N-acetyl-D-glucosamine residues.